{
  "term_id": "GO:0004984",
  "gene_symbol": "OR1J2",
  "gene_name": "Olfactory receptor 1J2",
  "gene": "UniProtKB:Q8NGS2",
  "term_label": "olfactory receptor activity"
}